{
  "gene": "UniProtKB:Q9P0T4",
  "term_label": "DNA-binding transcription factor activity",
  "gene_name": "Zinc finger protein 581",
  "term_id": "GO:0003700",
  "gene_symbol": "ZNF581"
}